{
  "term_label": "negative regulation of transcription by RNA polymerase II",
  "gene": "UniProtKB:P37231",
  "gene_symbol": "PPARG",
  "gene_name": "Peroxisome proliferator-activated receptor gamma",
  "term_id": "GO:0000122"
}